zonula adherens [GO:0005915] (cellular component) Also known as: adhesion belt, belt desmosome, intermediate junction, zonula adhaerens Sources: ISBN:0815316208 Relationships: is a type of adherens junction [GO:0005912]; is part of apical junction complex [GO:0043296] Definition: A cell-cell adherens junction which forms a continuous belt near the apex of epithelial cells. Subtypes: puncta adhaerentia [GO:0044288]